translation at presynapse, modulating chemical synaptic transmission [GO:0140237] (biological process) Relationships: is a type of translation at presynapse [GO:0140236]; regulates chemical synaptic transmission [GO:0007268] Definition: Translation that occurs at the presynapse, and that modulates chemical synaptic transmission. Note: Note that this term was created for the SynGO project, and will be obsoleted when the SynGO annotations are made in Noctua. References: PMID:27321671